{
  "term_label": "external side of plasma membrane",
  "term_id": "GO:0009897",
  "gene": "UniProtKB:P14207",
  "gene_name": "Folate receptor beta",
  "gene_symbol": "FOLR2"
}